regulation of growth rate [GO:0040009] (biological process) Note: Note that this term and its definition depart from the usual conventions for GO 'regulation' process terms; regulation of rate is not usually distinguished from regulation of extent or frequency, but it makes sense to do so for growth regulation. Sources: GOC:mah Definition: Any process that modulates the rate of growth of all or part of an organism. Relationships: is a type of regulation of growth [GO:0040008] Subtypes: positive regulation of growth rate [GO:0040010], negative regulation of growth rate [GO:0045967]